positive regulation of mitotic sister chromatid segregation [GO:0062033] (biological process) Definition: Any process that starts or increases the frequency, rate or extent of sister chromatid segregation during mitosis. Subtypes: negative regulation of mitotic spindle assembly checkpoint signaling [GO:0140499], GO:1902846 References: PMID:12773390 Relationships: is a type of regulation of mitotic sister chromatid segregation [GO:0033047]; is a type of positive regulation of chromosome segregation [GO:0051984]; is_a GO:2001252; positively regulates GO:0000070